uroporphyrin-III C-methyltransferase activity [GO:0004851] (molecular function) Also known as: CobA, CysG, S-adenosyl-L-methionine-dependent uroporphyrinogen III methylase activity, S-adenosyl-L-methionine:uroporphyrin-III C-methyltransferase activity, S-adenosyl-L-methionine:uroporphyrinogen-III C-methyltransferase activity, SUMT activity, SirA, adenosylmethionine-uroporphyrinogen III methyltransferase activity, urogen III methylase activity, uroporphyrinogen III methylase activity, uroporphyrinogen methyltransferase activity, uroporphyrinogen-III C-methyltransferase activity, uroporphyrinogen-III methylase activity, uroporphyrinogen-III methyltransferase activity Sources: EC:2.1.1.107 Definition: Catalysis of the reaction: 2 S-adenosyl-L-methionine + uroporphyrin III = 2 S-adenosyl-L-homocysteine + precorrin-2. Relationships: is a type of C-methyltransferase activity [GO:0008169]; is a type of S-adenosylmethionine-dependent methyltransferase activity [GO:0008757]